{
  "gene": "UniProtKB:Q9HB58",
  "term_id": "GO:0005634",
  "gene_name": "Sp110 nuclear body protein",
  "gene_symbol": "SP110",
  "term_label": "nucleus"
}